guanosine tetraphosphate metabolic process [GO:0015969] (biological process) Relationships: is a type of purine ribonucleotide metabolic process [GO:0009150]; is a type of GO:0034035 Definition: The chemical reactions and pathways involving guanine tetraphosphate (5'-ppGpp-3'), a derivative of guanine riboside with four phosphates. Subtypes: GO:0015970, GO:0015971 Sources: GOC:ai Also known as: guanosine tetraphosphate (5'-ppGpp-3') metabolic process, guanosine tetraphosphate (5'-ppGpp-3') metabolism, guanosine tetraphosphate metabolism